{
  "gene_name": "Large subunit GTPase 1 homolog",
  "gene_symbol": "LSG1",
  "term_id": "GO:0000054",
  "term_label": "ribosomal subunit export from nucleus",
  "gene": "UniProtKB:Q9H089"
}